{
  "gene_symbol": "ETFBKMT",
  "gene": "UniProtKB:Q8IXQ9",
  "gene_name": "Electron transfer flavoprotein beta subunit lysine methyltransferase",
  "term_id": "GO:1904736",
  "term_label": "negative regulation of fatty acid beta-oxidation using acyl-CoA dehydrogenase"
}